{
  "gene_symbol": "MTFR1",
  "gene": "UniProtKB:Q15390",
  "term_id": "GO:0009060",
  "term_label": "aerobic respiration",
  "gene_name": "Mitochondrial fission regulator 1"
}